{
  "term_id": "GO:0003723",
  "term_label": "RNA binding",
  "gene_name": "Heterogeneous nuclear ribonucleoprotein F",
  "gene_symbol": "HNRNPF",
  "gene": "UniProtKB:P52597"
}